regulation of somatic muscle development [GO:0062223] (biological process) References: PMID:16643882, PMID:25758712 Subtypes: positive regulation of somatic muscle development [GO:0062224], negative regulation of somatic muscle development [GO:0062225], GO:0062226, regulation of larval somatic muscle development [GO:0062229] Definition: Any process that regulates the rate, frequency or extent of somatic muscle development. Relationships: is a type of regulation of developmental process [GO:0050793]; regulates GO:0007525